{
  "gene_name": "G2_M phase-specific E3 ubiquitin-protein ligase",
  "term_label": "nucleus",
  "gene": "UniProtKB:Q7L622",
  "gene_symbol": "G2E3",
  "term_id": "GO:0005634"
}